{
  "gene_name": "Condensin-2 complex subunit G2",
  "term_id": "UNKNOWN:0001",
  "term_label": "Unknown molecular function",
  "gene": "UniProtKB:Q86XI2",
  "gene_symbol": "NCAPG2"
}